{
  "gene_symbol": "OCA2",
  "term_id": "GO:0033162",
  "term_label": "melanosome membrane",
  "gene_name": "P protein",
  "gene": "UniProtKB:Q04671"
}